{
  "gene_symbol": "BICRA",
  "term_id": "UNKNOWN:0001",
  "gene_name": "BRD4-interacting chromatin-remodeling complex-associated protein",
  "term_label": "Unknown molecular function",
  "gene": "UniProtKB:Q9NZM4"
}